positive regulation of metanephric mesenchymal cell migration [GO:2000591] (biological process) Definition: Any process that activates or increases the frequency, rate or extent of metanephric mesenchymal cell migration. Sources: GOC:mtg_kidney_jan10, GOC:obol, GOC:yaf Subtypes: positive regulation of metanephric mesenchymal cell migration by platelet-derived growth factor receptor-beta signaling pathway [GO:0035793] Also known as: positive regulation of metanephric mesenchyme chemotaxis Relationships: is a type of GO:0030335; is a type of regulation of metanephric mesenchymal cell migration [GO:2000589]; positively regulates metanephric mesenchymal cell migration [GO:0035789]